{
  "term_id": "GO:0005634",
  "gene": "UniProtKB:P40425",
  "gene_symbol": "PBX2",
  "term_label": "nucleus",
  "gene_name": "Pre-B-cell leukemia transcription factor 2"
}